glutamine family amino acid metabolic process [GO:0009064] (BP) Definition: The chemical reactions and pathways involving amino acids of the glutamine family, comprising arginine, glutamate, glutamine and proline. Subtypes: GO:0006527, glutamate metabolic process [GO:0006536], GO:0006541, proline metabolic process [GO:0006560], glutamine family amino acid biosynthetic process [GO:0009084], GO:0033388 Sources: GOC:ai Relationships: is a type of L-amino acid metabolic process [GO:0170033]; is a type of proteinogenic amino acid metabolic process [GO:0170039] Also known as: glutamine family amino acid metabolism